BRISC complex [GO:0070552] (cellular component) Relationships: is a type of GO:0140513 References: PMID:19214193 Sources: GOC:mah Definition: A protein complex that contains the FAM175B/ABRO1, BRCC3/BRCC36, BRE/BRCC45 and MERIT40/NBA1 proteins, and specifically cleaves K63-linked polyubiquitin chains.